{
  "gene_symbol": "NODAL",
  "gene": "UniProtKB:Q96S42",
  "term_label": "cell differentiation",
  "gene_name": "Nodal homolog",
  "term_id": "GO:0030154"
}